{
  "gene_name": "Histone H1.8",
  "gene_symbol": "H1-8",
  "gene": "UniProtKB:Q8IZA3",
  "term_label": "negative regulation of DNA recombination",
  "term_id": "GO:0045910"
}